leukemia inhibitory factor signaling pathway [GO:0048861] (biological process) Relationships: is a type of GO:0007167 Sources: GOC:devbiol, GOC:signaling Also known as: leukemia inhibitory factor signalling pathway Subtypes: leukemia inhibitory factor signaling pathway involved in forebrain neuron fate commitment [GO:0022025] Definition: The series of molecular signals initiated by the binding of a leukemia inhibitory factor to its receptor on the surface of a target cell, and ending with the regulation of a downstream cellular process, e.g. transcription.